{
  "gene": "UniProtKB:Q6UXZ0",
  "gene_name": "Transmembrane and immunoglobulin domain-containing protein 1",
  "gene_symbol": "TMIGD1",
  "term_id": "UNKNOWN:0001",
  "term_label": "Unknown molecular function"
}